{
  "gene_symbol": "OCM",
  "term_id": "GO:0005509",
  "gene_name": "Oncomodulin-1",
  "gene": "UniProtKB:P0CE72",
  "term_label": "calcium ion binding"
}